{
  "gene_symbol": "BROX",
  "term_label": "Unknown biological process",
  "gene_name": "BRO1 domain-containing protein BROX",
  "term_id": "UNKNOWN:0002",
  "gene": "UniProtKB:Q5VW32"
}